positive regulation of DNA binding [GO:0043388] (biological process) Definition: Any process that increases the frequency, rate or extent of DNA binding. DNA binding is any process in which a gene product interacts selectively with DNA (deoxyribonucleic acid). Sources: GOC:dph, GOC:jl, GOC:tb Also known as: up regulation of DNA binding, up-regulation of DNA binding, upregulation of DNA binding, activation of DNA binding, stimulation of DNA binding Relationships: is a type of positive regulation of binding [GO:0051099]; is a type of regulation of DNA binding [GO:0051101]; positively regulates DNA binding [GO:0003677] Subtypes: positive regulation of transcription regulatory region DNA binding [GO:2000679]